{
  "term_id": "UNKNOWN:0003",
  "gene_symbol": "NKAIN1",
  "gene_name": "Sodium_potassium-transporting ATPase subunit beta-1-interacting protein 1",
  "term_label": "Unknown cellular component",
  "gene": "UniProtKB:Q4KMZ8"
}